sequestering of TGFbeta from receptor via TGFbeta binding [GO:0038105] (biological process) Note: This term is for annotation of gene products that bind to TGFbeta. For gene products that tether the TGFbeta-containing latency complex to the extracellular matrix, but do not necessarily bind TGF-beta directly, consider instead annotating to 'sequestering of TGFbeta in extracellular matrix ; GO:0035583'. Relationships: is a type of sequestering of extracellular ligand from receptor [GO:0035581] References: PMID:19855014 Sources: GOC:bf, GOC:signaling Also known as: extracellular sequestering of TGFbeta, extracellular sequestering of transforming growth factor-beta Definition: Binding to a transforming growth factor-beta (TGFbeta) protein in the extracellular region, and inhibiting TGFbeta signaling by preventing TGFbeta from binding to its cell surface receptor.